venom-mediated perturbation of pH-gated ion channel activity [GO:0044733] (biological process) Also known as: envenomation resulting in modulation of ASIC channel activity in other organism, envenomation resulting in modulation of acid-sensing ion channel activity in another organism, envenomation resulting in modulation of acid-sensing ion channel activity in other organism, venom-mediated perturbation of acid-sensing ion channel activity Relationships: is a type of venom-mediated perturbation of ion channel activity [GO:0044560] Subtypes: GO:0044734, venom-mediated inhibition of pH-gated ion channel activity [GO:0044735] References: PMID:23034652 Sources: GOC:fj, GOC:jl Definition: A process in which an organism alters or subverts the activity of a pH-gated (also known as acid-sensing ion channel (ASIC)) in another organism via the action of a venom.